{
  "term_id": "UNKNOWN:0002",
  "gene_symbol": "ARHGEF38",
  "term_label": "Unknown biological process",
  "gene_name": "Rho guanine nucleotide exchange factor 38",
  "gene": "UniProtKB:Q9NXL2"
}